{
  "term_id": "GO:0005764",
  "gene_name": "Mammalian ependymin-related protein 1",
  "term_label": "lysosome",
  "gene": "UniProtKB:Q9UM22",
  "gene_symbol": "EPDR1"
}